peptidyl-prolyl cis-trans isomerase activity [GO:0003755] (molecular function) Also known as: cis-trans proline isomerase activity, FK506-sensitive peptidyl-prolyl cis-trans isomerase, cyclophilin-type peptidyl-prolyl cis-trans isomerase activity, juglone-sensitive cis-trans proline isomerase activity, juglone-sensitive peptidyl-prolyl cis-trans isomerase activity, PPIase activity, cyclophilin activity, immunophilin, parvulin, peptide bond isomerase activity, peptidyl-prolyl isomerase B reaction, peptidylproline cis-trans-isomerase activity, peptidylprolyl cis-trans isomerase activity, peptidylprolyl isomerase activity, rotamase activity Definition: Catalysis of the reaction: peptidyl-proline (omega=180) = peptidyl-proline (omega=0). Subtypes: RNA polymerase II CTD heptapeptide repeat peptidyl-prolyl isomerase activity [GO:0140838] Sources: EC:5.2.1.8 Relationships: is a type of cis-trans isomerase activity [GO:0016859]; is a type of catalytic activity, acting on a protein [GO:0140096]